{
  "term_label": "synapse organization",
  "gene": "UniProtKB:Q9UBF9",
  "gene_symbol": "MYOT",
  "gene_name": "Myotilin",
  "term_id": "GO:0050808"
}